aerobactin synthase activity [GO:0050565] (molecular function) Sources: RHEA:32167 Also known as: citrate:6-N-acetyl-6-N-hydroxy-L-lysine ligase (ADP-forming), citrate:N6-acetyl-N6-hydroxy-L-lysine ligase (ADP-forming) Relationships: is a type of acid-amino acid ligase activity [GO:0016881] Definition: Catalysis of the reaction: ATP + N2-citryl-N6-acetyl-N6-hydroxy-L-lysine + N6-acetyl-N6-hydroxy-L-lysine = aerobactin + AMP + diphosphate + H+.